{
  "term_id": "GO:0000506",
  "term_label": "glycosylphosphatidylinositol-N-acetylglucosaminyltransferase (GPI-GnT) complex",
  "gene_name": "Phosphatidylinositol N-acetylglucosaminyltransferase subunit A",
  "gene": "UniProtKB:P37287",
  "gene_symbol": "PIGA"
}